{
  "gene_name": "Serine_threonine-protein kinase Kist",
  "gene": "UniProtKB:Q8TAS1",
  "term_id": "GO:0043021",
  "term_label": "ribonucleoprotein complex binding",
  "gene_symbol": "UHMK1"
}